{
  "gene_symbol": "UBE2G2",
  "gene_name": "Ubiquitin-conjugating enzyme E2 G2",
  "term_id": "GO:0005783",
  "term_label": "endoplasmic reticulum",
  "gene": "UniProtKB:P60604"
}